{
  "gene_symbol": "PRKDC",
  "gene": "UniProtKB:P78527",
  "gene_name": "DNA-dependent protein kinase catalytic subunit",
  "term_label": "telomere maintenance",
  "term_id": "GO:0000723"
}